cellular response to auxin stimulus [GO:0071365] (biological process) Relationships: is a type of response to auxin [GO:0009733]; is a type of GO:0032870 Subtypes: cellular response to indolebutyric acid stimulus [GO:0071366] Sources: GOC:mah Definition: Any process that results in a change in state or activity of a cell (in terms of movement, secretion, enzyme production, gene expression, etc.) as a result of an auxin stimulus.